{
  "gene_symbol": "TMEM43",
  "term_label": "nuclear membrane organization",
  "gene": "UniProtKB:Q9BTV4",
  "term_id": "GO:0071763",
  "gene_name": "Transmembrane protein 43"
}